{
  "term_id": "GO:0005737",
  "term_label": "cytoplasm",
  "gene": "UniProtKB:Q2M3C7",
  "gene_symbol": "SPHKAP",
  "gene_name": "A-kinase anchor protein SPHKAP"
}